{
  "term_id": "GO:0006357",
  "gene": "UniProtKB:Q01543",
  "gene_symbol": "FLI1",
  "gene_name": "Friend leukemia integration 1 transcription factor",
  "term_label": "regulation of transcription by RNA polymerase II"
}